low-density lipoprotein particle [GO:0034362] (cellular component) Relationships: is a type of plasma lipoprotein particle [GO:0034358] Sources: GOC:BHF, GOC:expert_pt, GOC:mah, GOC:rl Definition: A lipoprotein particle, rich in cholesterol esters and low in triglycerides that is typically composed of APOB100 and APOE and has a density of 1.02-1.06 g/ml and a diameter of between 20-25 nm. LDL particles are formed from VLDL particles (via IDL) by the loss of triglyceride and gain of cholesterol ester. They transport endogenous cholesterol (and to some extent triglycerides) from peripheral tissues back to the liver. Also known as: LDL complex, LDL particle, low-density lipoprotein complex